{
  "term_label": "cytosol",
  "gene": "UniProtKB:P29558",
  "gene_symbol": "RBMS1",
  "gene_name": "RNA-binding motif, single-stranded-interacting protein 1",
  "term_id": "GO:0005829"
}